{
  "gene": "UniProtKB:Q96IC2",
  "gene_symbol": "REXO5",
  "term_label": "exonuclease activity",
  "gene_name": "RNA exonuclease 5",
  "term_id": "GO:0004527"
}